follicle cell of egg chamber migration [GO:0007297] (biological process) Definition: The directed movement of an ovarian follicle cell that takes place during oogenesis. During egg chamber formation, follicle cells migrate to envelop the germ-line cysts and move in between cysts. At stage 10B, follicle cells migrate centripetally between the nurse cells and the oocyte, enclosing the anterior of the egg. An example of this is found in Drosophila melanogaster. References: PMID:10822261 Sources: GOC:mtg_sensu Also known as: follicle cell migration Relationships: is a type of epithelial cell migration [GO:0010631]; is part of follicle cell of egg chamber development [GO:0030707] Subtypes: GO:0007298, centripetally migrating follicle cell migration [GO:0060269], main body follicle cell migration [GO:0060270]